late endosome [GO:0005770] (cellular component) Definition: A prelysosomal endocytic organelle differentiated from early endosomes by lower lumenal pH and different protein composition. Late endosomes are more spherical than early endosomes and are mostly juxtanuclear, being concentrated near the microtubule organizing center. References: PMID:11964142, PMID:2557062 Sources: NIF_Subcellular:nlx_subcell_20090702 Also known as: PVC, prevacuolar compartment Relationships: is a type of endosome [GO:0005768] Subtypes: GO:0005771